{
  "gene": "UniProtKB:Q9BVL4",
  "term_id": "UNKNOWN:0002",
  "gene_name": "Protein adenylyltransferase SelO, mitochondrial",
  "term_label": "Unknown biological process",
  "gene_symbol": "SELENOO"
}